regulation of uterine smooth muscle relaxation [GO:1900719] (biological process) Also known as: regulation of smooth muscle relaxation of the uterus Sources: GOC:TermGenie Subtypes: negative regulation of uterine smooth muscle relaxation [GO:1900720], positive regulation of uterine smooth muscle relaxation [GO:1900721] Relationships: is_a regulation of relaxation of smooth muscle [GO:1901080]; RO_0002211 GO:0044558 Definition: Any process that modulates the frequency, rate or extent of uterine smooth muscle relaxation.